growth plate cartilage chondrocyte morphogenesis [GO:0003429] (biological process) Sources: GOC:ascb_2009, GOC:dph, GOC:tb Relationships: is a type of chondrocyte morphogenesis involved in endochondral bone morphogenesis [GO:0003414]; is a type of growth plate cartilage morphogenesis [GO:0003422]; is part of growth plate cartilage chondrocyte differentiation [GO:0003418] Definition: The process in which the structures of a chondrocyte in the growth plate cartilage are generated and organized.